{
  "gene": "UniProtKB:Q2M5E4",
  "gene_symbol": "RGS21",
  "term_id": "GO:0045744",
  "term_label": "negative regulation of G protein-coupled receptor signaling pathway",
  "gene_name": "Regulator of G-protein signaling 21"
}